{
  "term_label": "semaphorin receptor binding",
  "term_id": "GO:0030215",
  "gene_name": "Semaphorin-5A",
  "gene_symbol": "SEMA5A",
  "gene": "UniProtKB:Q13591"
}